regulation of convergent extension involved in gastrulation [GO:1904103] (biological process) Definition: Any process that modulates the frequency, rate or extent of convergent extension involved in gastrulation. References: PMID:24892953 Sources: GOC:TermGenie, GOC:dph, GO_REF:0000058 Relationships: is_a GO:1905330; RO_0002211 convergent extension involved in gastrulation [GO:0060027] Subtypes: negative regulation of convergent extension involved in gastrulation [GO:1904104], positive regulation of convergent extension involved in gastrulation [GO:1904105], regulation of convergent extension involved in somitogenesis [GO:1904127], regulation of convergent extension involved in neural plate elongation [GO:1904130], regulation of convergent extension involved in rhombomere morphogenesis [GO:1904133], regulation of convergent extension involved in notochord morphogenesis [GO:1904136]